rRNA metabolic process [GO:0016072] (biological process) Sources: ISBN:0198506732 Definition: The chemical reactions and pathways involving rRNA, ribosomal RNA, a structural constituent of ribosomes. Subtypes: rRNA processing [GO:0006364], rRNA transcription [GO:0009303], GO:0016075 Also known as: rRNA metabolism Relationships: is a type of RNA metabolic process [GO:0016070]